establishment or maintenance of polarity of larval imaginal disc epithelium [GO:0016336] (biological process) Definition: Any cellular process that results in the specification, formation or maintenance of a polarized larval imaginal disc epithelium. Sources: GOC:jl, GOC:mah Subtypes: GO:0042251 Relationships: is a type of establishment or maintenance of cell polarity [GO:0007163]; is part of morphogenesis of larval imaginal disc epithelium [GO:0016335]